{
  "gene": "UniProtKB:P16444",
  "term_label": "plasma membrane",
  "gene_name": "Dipeptidase 1",
  "gene_symbol": "DPEP1",
  "term_id": "GO:0005886"
}